{
  "term_id": "UNKNOWN:0001",
  "gene_symbol": "GOLGA8IP",
  "term_label": "Unknown molecular function",
  "gene": "UniProtKB:A6NC78",
  "gene_name": "Putative golgin subfamily A member 8I"
}